{
  "gene_name": "tRNA N(3)-methylcytidine methyltransferase METTL2B",
  "term_label": "Unknown biological process",
  "gene_symbol": "METTL2B",
  "gene": "UniProtKB:Q6P1Q9",
  "term_id": "UNKNOWN:0002"
}